{
  "term_id": "GO:0046208",
  "gene_name": "Spermine oxidase",
  "term_label": "spermine catabolic process",
  "gene": "UniProtKB:Q9NWM0",
  "gene_symbol": "SMOX"
}